calmodulin-lysine N-methyltransferase activity [GO:0018025] (molecular function) Definition: Catalysis of the reaction: S-adenosyl-L-methionine + calmodulin L-lysine = S-adenosyl-L-homocysteine + calmodulin N6-methyl-L-lysine. Relationships: is a type of protein-lysine N-methyltransferase activity [GO:0016279] Sources: EC:2.1.1.60 Also known as: S-adenosyl-L-methionine:calmodulin-L-lysine 6-N-methyltransferase activity, S-adenosyl-L-methionine:calmodulin-L-lysine N6-methyltransferase activity, S-adenosylmethionine:calmodulin (lysine) N-methyltransferase activity